{
  "gene": "UniProtKB:A8MVU1",
  "term_label": "superoxide-generating NADPH oxidase activator activity",
  "gene_name": "Putative neutrophil cytosol factor 1C",
  "term_id": "GO:0016176",
  "gene_symbol": "NCF1C"
}